{
  "term_label": "cell morphogenesis",
  "term_id": "GO:0000902",
  "gene_symbol": "CDH3",
  "gene_name": "Cadherin-3",
  "gene": "UniProtKB:P22223"
}